{
  "gene": "UniProtKB:Q9BT04",
  "term_id": "UNKNOWN:0001",
  "gene_symbol": "FUZ",
  "term_label": "Unknown molecular function",
  "gene_name": "Protein fuzzy homolog"
}